{
  "gene": "UniProtKB:A0A0U1RRA0",
  "term_label": "Unknown molecular function",
  "gene_name": "Putative transmembrane protein ZNF593OS",
  "gene_symbol": "ZNF593OS",
  "term_id": "UNKNOWN:0001"
}